{
  "gene": "UniProtKB:Q9H0K4",
  "gene_name": "Radial spoke head protein 6 homolog A",
  "term_id": "GO:0003341",
  "gene_symbol": "RSPH6A",
  "term_label": "cilium movement"
}